cytochrome P450 dependent ent-sandaracopimaradiene 3-hydroxylase activity [GO:0102596] (molecular function) Sources: EC:1.14.14.70, GOC:pz Definition: Catalysis of the reaction: ent-sandaracopimara-8(14),15-diene + NADPH + H+ + O2 = ent-sandaracopimaradien-3beta-ol + NADP + H2O. Relationships: is a type of GO:0016709